{
  "term_id": "UNKNOWN:0002",
  "term_label": "Unknown biological process",
  "gene": "UniProtKB:Q5MJ07",
  "gene_symbol": "SPANXN5",
  "gene_name": "Sperm protein associated with the nucleus on the X chromosome N5"
}